{
  "term_label": "Unknown molecular function",
  "term_id": "UNKNOWN:0001",
  "gene_name": "T cell receptor beta variable 14",
  "gene": "UniProtKB:A0A5B0",
  "gene_symbol": "TRBV14"
}